suramin binding [GO:0043924] (molecular function) Sources: GOC:jl, Wikipedia:Suramin Also known as: Germanin binding Definition: Binding to suramin, a naphthalenesulfonic acid compound which is used in the treatment of diseases caused by trypanosomes and worms. Relationships: is_a amide binding [GO:0033218]; is a type of anion binding [GO:0043168]; is a type of GO:0043177; is_a sulfur compound binding [GO:1901681]